epsilon-caprolactam lactamase activity [GO:0018752] (molecular function) Relationships: is a type of GO:0016812 Sources: UM-BBD_reactionID:r0448 Definition: Catalysis of the reaction: epsilon-caprolactam + H2O = H+ + 6-aminohexanoate.